{
  "gene_symbol": "FAM87A",
  "gene": "UniProtKB:P0C7U9",
  "term_id": "UNKNOWN:0002",
  "gene_name": "Protein FAM87A",
  "term_label": "Unknown biological process"
}